{
  "term_id": "GO:0001764",
  "gene": "UniProtKB:Q8NEY1",
  "gene_name": "Neuron navigator 1",
  "term_label": "neuron migration",
  "gene_symbol": "NAV1"
}